effector-mediated induction of cell cycle reactivation in host [GO:0141017] (biological process) Definition: A symbiont process in which a molecule secreted by the symbiont reactivates the host cell cycle, resulting in DNA synthesis and host cell division, and contributing to vegetative tumor formation. References: PMID:25888589 Relationships: is a type of effector-mediated perturbation of host process by symbiont [GO:0140418]; is part of symbiont-mediated induction of tumor or growth in host [GO:0051819]